{
  "gene_symbol": "PCSK1",
  "term_label": "membrane",
  "term_id": "GO:0016020",
  "gene_name": "Neuroendocrine convertase 1",
  "gene": "UniProtKB:P29120"
}